{
  "gene_name": "Immunoglobulin lambda joining 6 (Fragment)",
  "term_label": "Unknown cellular component",
  "gene_symbol": "IGLJ6",
  "term_id": "UNKNOWN:0003",
  "gene": "UniProtKB:A0A0A0MT93"
}